{
  "gene_symbol": "BTBD8",
  "term_label": "Unknown biological process",
  "gene_name": "BTB_POZ domain-containing protein 8",
  "gene": "UniProtKB:Q5XKL5",
  "term_id": "UNKNOWN:0002"
}